{
  "gene_symbol": "RBMY1F",
  "gene": "UniProtKB:Q15415",
  "gene_name": "RNA-binding motif protein, Y chromosome, family 1 member F_J",
  "term_label": "spliceosomal complex",
  "term_id": "GO:0005681"
}